regulation of the force of heart contraction by cardiac conduction [GO:0086092] (biological process) Sources: GOC:BHF, GOC:mtg_cardiac_conduct_nov11 Relationships: is_a GO:0002026; is a type of cardiac conduction [GO:0061337] Definition: A cardiac conduction process that modulates the extent of heart contraction, changing the force with which blood is propelled.